{
  "gene_symbol": "RNF168",
  "term_id": "GO:0031491",
  "term_label": "nucleosome binding",
  "gene": "UniProtKB:Q8IYW5",
  "gene_name": "E3 ubiquitin-protein ligase RNF168"
}